{
  "term_id": "GO:0061630",
  "term_label": "ubiquitin protein ligase activity",
  "gene_symbol": "TRIM43B",
  "gene": "UniProtKB:A6NCK2",
  "gene_name": "Tripartite motif-containing protein 43B"
}